cytoplasmic translational termination [GO:0002184] (biological process) Relationships: is a type of translational termination [GO:0006415]; is part of cytoplasmic translation [GO:0002181]; occurs in cytosol [GO:0005829] Sources: GOC:hjd Definition: The process resulting in the release of a polypeptide chain from the ribosome in the cytoplasm, usually in response to a termination codon. Regulation: regulated by regulation of cytoplasmic translational termination [GO:1990580]